colicin transmembrane transporter activity [GO:0042912] (molecular function) Subtypes: group A colicin transmembrane transporter activity [GO:0042913] Definition: Enables the transfer of a colicin from one side of a membrane to the other. Colicins are a group of antibiotics produced by E. coli and related species that are encoded by a group of naturally occurring plasmids, e.g. Col E1. References: PMID:17347522 Sources: GOC:jl, GOC:mtg_transport, ISBN:0815340729 Relationships: is a type of bacteriocin transmembrane transporter activity [GO:0022885]